{
  "gene_name": "Glutathione peroxidase 7",
  "term_id": "GO:0034599",
  "gene_symbol": "GPX7",
  "gene": "UniProtKB:Q96SL4",
  "term_label": "cellular response to oxidative stress"
}